positive regulation of telomeric loop formation [GO:1904420] (BP) References: PMID:22579284 Sources: GOC:BHF, GOC:BHF_telomere, GOC:TermGenie, GOC:nc, GO_REF:0000058 Also known as: positive regulation of t-loop biosynthesis, positive regulation of t-loop formation, up regulation of t-loop biosynthesis, up regulation of t-loop formation, up regulation of telomeric loop formation, up-regulation of t-loop biosynthesis, up-regulation of t-loop formation, up-regulation of telomeric loop formation, upregulation of t-loop biosynthesis, upregulation of t-loop formation, upregulation of telomeric loop formation, activation of t-loop biosynthesis, activation of t-loop formation, activation of telomeric loop formation Relationships: is a type of positive regulation of telomere maintenance [GO:0032206]; is a type of regulation of telomeric loop formation [GO:1904418]; positively regulates telomeric loop formation [GO:0031627] Definition: Any process that activates or increases the frequency, rate or extent of telomeric loop formation.